behavioral defense response [GO:0002209] (biological process) Sources: GOC:add, GO_REF:0000022 Subtypes: GO:0001662, behavioral defense response to insect [GO:0002211], GO:0002212 Definition: A behavioral response seeking to protect an organism from an perceived external threat to that organism. Relationships: is a type of defense response [GO:0006952]; is a type of behavior [GO:0007610] Also known as: behavioural defense response